{
  "gene_name": "Supervillin",
  "gene_symbol": "SVIL",
  "gene": "UniProtKB:O95425",
  "term_id": "GO:0051015",
  "term_label": "actin filament binding"
}